dicarboxylic acid transport [GO:0006835] (biological process) Definition: The directed movement of dicarboxylic acids into, out of or within a cell, or between cells, by means of some agent such as a transporter or pore. Subtypes: glutamate secretion [GO:0014047], bilirubin transport [GO:0015723], GO:0015740, alpha-ketoglutarate transport [GO:0015742], p-aminobenzoyl-glutamate transport [GO:0015814], GO:0015884, 5-formyltetrahydrofolate transport [GO:0015885], oxalate transport [GO:0019532], isopropylmalate transport [GO:0034659], aldarate transmembrane transport [GO:0042869], L-glutamate import [GO:0051938], GO:0051958, glutamate transmembrane import into vacuole [GO:0090454], malonic acid transport [GO:1900752], quinolinic acid transmembrane transport [GO:1903222], GO:1990551 Sources: GOC:krc Also known as: sodium:dicarboxylate transport Relationships: is a type of carboxylic acid transport [GO:0046942]